{
  "gene": "UniProtKB:Q8NFZ8",
  "gene_symbol": "CADM4",
  "term_label": "regulation of Rac protein signal transduction",
  "gene_name": "Cell adhesion molecule 4",
  "term_id": "GO:0035020"
}